{
  "term_label": "Unknown cellular component",
  "gene_symbol": "CCDC89",
  "gene": "UniProtKB:Q8N998",
  "term_id": "UNKNOWN:0003",
  "gene_name": "Coiled-coil domain-containing protein 89"
}